{
  "term_label": "aryl hydrocarbon receptor complex",
  "gene_name": "Basic helix-loop-helix ARNT-like protein 2",
  "gene_symbol": "BMAL2",
  "term_id": "GO:0034751",
  "gene": "UniProtKB:Q8WYA1"
}